{
  "gene_name": "Uncharacterized protein",
  "term_id": "UNKNOWN:0002",
  "term_label": "Unknown biological process",
  "gene": "UniProtKB:A0A7I2V6D3",
  "gene_symbol": "A0A7I2V6D3"
}